{
  "gene": "UniProtKB:Q99678",
  "gene_symbol": "GPR20",
  "gene_name": "G-protein coupled receptor 20",
  "term_label": "G protein-coupled receptor activity",
  "term_id": "GO:0004930"
}